{
  "term_label": "Unknown molecular function",
  "gene": "UniProtKB:Q92610",
  "gene_name": "Zinc finger protein 592",
  "gene_symbol": "ZNF592",
  "term_id": "UNKNOWN:0001"
}